{
  "term_label": "taste receptor activity",
  "gene_name": "Free fatty acid receptor 4",
  "term_id": "GO:0008527",
  "gene_symbol": "FFAR4",
  "gene": "UniProtKB:Q5NUL3"
}